{
  "gene": "UniProtKB:Q13905",
  "gene_symbol": "RAPGEF1",
  "term_id": "GO:0007265",
  "gene_name": "Rap guanine nucleotide exchange factor 1",
  "term_label": "Ras protein signal transduction"
}